{
  "term_label": "DNA-binding transcription factor activity, RNA polymerase II-specific",
  "gene_symbol": "SMAD1",
  "gene_name": "Mothers against decapentaplegic homolog 1",
  "term_id": "GO:0000981",
  "gene": "UniProtKB:Q15797"
}